{
  "gene_symbol": "PRADC1",
  "gene": "UniProtKB:Q9BSG0",
  "term_label": "Unknown cellular component",
  "term_id": "UNKNOWN:0003",
  "gene_name": "Protease-associated domain-containing protein 1"
}